{
  "gene": "UniProtKB:Q8NHY3",
  "term_id": "GO:0035371",
  "gene_symbol": "GAS2L2",
  "term_label": "microtubule plus-end",
  "gene_name": "GAS2-like protein 2"
}